2-phosphosulfolactate phosphatase activity [GO:0050532] (molecular function) Definition: Catalysis of the reaction: (2R)-O-phospho-3-sulfolactate + H2O = (R)-3-sulfolactate + phosphate. Sources: EC:3.1.3.71, RHEA:23416 Also known as: 2-phosphosulpholactate phosphatase activity, (2R)-phosphosulfolactate phosphohydrolase activity, (R)-2-phospho-3-sulfolactate phosphohydrolase activity, ComB phosphatase activity Relationships: is a type of GO:0016791